transcription-dependent tethering of RNA polymerase II gene DNA at nuclear periphery [GO:0000972] (biological process) Subtypes: post-transcriptional tethering of RNA polymerase II gene DNA at nuclear periphery [GO:0000973] Definition: The chromosome organization process in which the DNA sequence containing a gene transcribed by RNA polymerase II is maintained in a specific location at the nuclear periphery. In S. cerevisiae, this process involves cis-acting DNA sequences such as the TATA box and upstream activating sequence (UAS) elements, trans-acting transcriptional activators, and also the 3'-UTR of the transcript. Relationships: is a type of chromosome organization [GO:0051276] References: PMID:18614049 Sources: GOC:krc